{
  "term_id": "GO:0004843",
  "gene_name": "OTU domain-containing protein 1",
  "gene_symbol": "OTUD1",
  "term_label": "cysteine-type deubiquitinase activity",
  "gene": "UniProtKB:Q5VV17"
}